{
  "gene_name": "Protein O-glucosyltransferase 2",
  "term_label": "endomembrane system",
  "gene": "UniProtKB:Q6UW63",
  "gene_symbol": "POGLUT2",
  "term_id": "GO:0012505"
}